blood vessel endothelial cell delamination [GO:0097497] (biological process) Subtypes: blood vessel endothelial cell delamination involved in blood vessel lumen ensheathment [GO:1902354] Definition: The process of negative regulation of cell adhesion that results in blood vessel endothelial cells splitting off from an existing endothelial sheet. Relationships: is a type of delamination [GO:0060232] References: PMID:23698350 Sources: GOC:dgh